{
  "gene_name": "Golgin subfamily A member 8M",
  "term_id": "GO:0005801",
  "gene": "UniProtKB:H3BSY2",
  "gene_symbol": "GOLGA8M",
  "term_label": "cis-Golgi network"
}